{
  "gene": "UniProtKB:A0A0G2JMM0",
  "gene_symbol": "LOC128966728",
  "gene_name": "Uncharacterized protein",
  "term_id": "GO:0002767",
  "term_label": "immune response-inhibiting cell surface receptor signaling pathway"
}